{
  "term_id": "GO:0005783",
  "gene": "UniProtKB:Q8IYP9",
  "gene_symbol": "ZDHHC23",
  "term_label": "endoplasmic reticulum",
  "gene_name": "Palmitoyltransferase ZDHHC23"
}